{
  "term_label": "proteasome-mediated ubiquitin-dependent protein catabolic process",
  "term_id": "GO:0043161",
  "gene_symbol": "PSMC4",
  "gene_name": "26S proteasome regulatory subunit 6B",
  "gene": "UniProtKB:P43686"
}